{
  "gene": "UniProtKB:Q9HBI5",
  "gene_name": "Centrosomal protein 15 kDa",
  "gene_symbol": "CEP15",
  "term_id": "UNKNOWN:0003",
  "term_label": "Unknown cellular component"
}